{
  "term_id": "GO:0005737",
  "gene": "UniProtKB:Q9ULV0",
  "gene_symbol": "MYO5B",
  "term_label": "cytoplasm",
  "gene_name": "Unconventional myosin-Vb"
}